{
  "term_id": "GO:0007548",
  "gene_symbol": "DMRT1",
  "gene": "UniProtKB:Q9Y5R6",
  "gene_name": "Doublesex- and mab-3-related transcription factor 1",
  "term_label": "sex differentiation"
}